{
  "gene": "UniProtKB:Q8TEY5",
  "term_id": "GO:0005634",
  "gene_symbol": "CREB3L4",
  "term_label": "nucleus",
  "gene_name": "Cyclic AMP-responsive element-binding protein 3-like protein 4"
}